{
  "gene_name": "Sialic acid-binding Ig-like lectin 6",
  "gene_symbol": "SIGLEC6",
  "gene": "UniProtKB:O43699",
  "term_id": "GO:0007155",
  "term_label": "cell adhesion"
}